nucleolus organizer region [GO:0005731] (cellular component) Also known as: NOR, nucleolus organiser region, nucleolus organizer complex References: PMID:14504406 Relationships: is a type of nucleolar chromatin [GO:0030874] Definition: A region of a chromosome where nucleoli form during interphase, and where genes encoding the largest rRNA precursor transcript are tandemly arrayed.